{
  "term_label": "negative regulation of gene expression, epigenetic",
  "gene_symbol": "SMYD5",
  "term_id": "GO:0045814",
  "gene": "UniProtKB:Q6GMV2",
  "gene_name": "Histone-lysine N-trimethyltransferase SMYD5"
}